maintenance of apical/basal cell polarity [GO:0035090] (biological process) Sources: GOC:bf Relationships: is a type of maintenance of cell polarity [GO:0030011]; is a type of establishment or maintenance of apical/basal cell polarity [GO:0035088] Subtypes: maintenance of epithelial cell apical/basal polarity [GO:0045199] Definition: Retaining the established polarization of a cell along its apical/basal axis.